ent-kaurene biosynthetic process [GO:0033332] (biological process) Also known as: ent-kaurene anabolism, ent-kaurene biosynthesis, ent-kaurene formation, ent-kaurene synthesis References: PMID:17064690 Sources: GOC:mah, MetaCyc:PWY-5032 Relationships: is a type of ent-kaurene metabolic process [GO:0033331]; is a type of terpene biosynthetic process [GO:0046246] Definition: The chemical reactions and pathways resulting in the formation of ent-kaurene. Ent-kaurene is a tetracyclic diterpenoid that is a precursor of several plant isoprenoids, including gibberellins.